{
  "gene": "UniProtKB:Q14994",
  "term_id": "GO:0000122",
  "gene_name": "Nuclear receptor subfamily 1 group I member 3",
  "gene_symbol": "NR1I3",
  "term_label": "negative regulation of transcription by RNA polymerase II"
}